undecaprenyl-phosphate 4-deoxy-4-formamido-L-arabinose transferase activity [GO:0099621] (MF) Definition: Catalysis of the reaction: UDP-4-deoxy-4-formamido-beta-L-arabinopyranose + ditrans,octacis-undecaprenyl phosphate = UDP + 4-deoxy-4-formamido-alpha-L-arabinopyranosyl ditrans,octacis-undecaprenyl phosphate. Also known as: Ara4FN transferase activity, undecaprenyl phosphate-L-Ara4FN transferase activity, undecaprenyl-phosphate Ara4FN transferase activity Relationships: is a type of pentosyltransferase activity [GO:0016763] References: PMID:11706007, PMID:15695810 Sources: GOC:al, GOC:dos